negative regulation of thymocyte aggregation [GO:2000399] (biological process) Relationships: is a type of GO:1903038; is a type of GO:2000398; RO_0002212 GO:0071594 Sources: GOC:BHF, GOC:mah Definition: Any process that stops, prevents or reduces the frequency, rate or extent of thymocyte aggregation. Also known as: negative regulation of T cell precursor aggregation, negative regulation of immature T-lymphocyte aggregation, negative regulation of thymic lymphocyte aggregation, negative regulation of immature T cell aggregation, negative regulation of immature T-cell aggregation